{
  "gene_name": "Large neutral amino acids transporter small subunit 1",
  "term_id": "GO:0015179",
  "gene_symbol": "SLC7A5",
  "gene": "UniProtKB:Q01650",
  "term_label": "L-amino acid transmembrane transporter activity"
}